{
  "term_id": "GO:0005783",
  "gene": "UniProtKB:P30101",
  "gene_symbol": "PDIA3",
  "gene_name": "Protein disulfide-isomerase A3",
  "term_label": "endoplasmic reticulum"
}